{
  "gene": "UniProtKB:Q8TAQ5",
  "term_label": "DNA-binding transcription factor activity, RNA polymerase II-specific",
  "term_id": "GO:0000981",
  "gene_symbol": "ZNF420",
  "gene_name": "Zinc finger protein 420"
}